oxidized base lesion DNA N-glycosylase activity [GO:0000702] (molecular function) Relationships: is a type of DNA N-glycosylase activity [GO:0019104] References: PMID:11554296 Sources: GOC:elh Definition: Catalysis of the removal of oxidized bases by cleaving the N-C1' glycosidic bond between the target damaged DNA base and the deoxyribose sugar. The reaction releases a free base and leaves an apurinic/apyrimidinic (AP) site. Subtypes: oxidized pyrimidine nucleobase lesion DNA N-glycosylase activity [GO:0000703], GO:0008534